{
  "gene": "UniProtKB:Q5JVS0",
  "term_id": "GO:0033120",
  "gene_name": "Intracellular hyaluronan-binding protein 4",
  "gene_symbol": "HABP4",
  "term_label": "positive regulation of RNA splicing"
}